PDX1-PBX1b-MRG1 complex [GO:0034978] (cellular component) Definition: A protein complex that contains the homeodomain proteins PDX1, PBX1b and MRG1 (MEIS2) and is involved in the transcriptional regulation of pancreatic acinar cell-specific genes. References: PMID:11279116, PMID:9710595 Also known as: acinar cell-specific C complex Relationships: is a type of nuclear protein-containing complex [GO:0140513]